{
  "gene_symbol": "A0A5F9ZHS0",
  "gene": "UniProtKB:A0A5F9ZHS0",
  "term_id": "UNKNOWN:0002",
  "gene_name": "Uncharacterized protein",
  "term_label": "Unknown biological process"
}